{
  "term_id": "UNKNOWN:0001",
  "gene_symbol": "SAMD13",
  "gene_name": "Sterile alpha motif domain-containing protein 13",
  "gene": "UniProtKB:Q5VXD3",
  "term_label": "Unknown molecular function"
}